{
  "gene_name": "Bridge-like lipid transfer protein family member 1",
  "gene": "UniProtKB:Q2LD37",
  "gene_symbol": "BLTP1",
  "term_id": "UNKNOWN:0001",
  "term_label": "Unknown molecular function"
}